{
  "term_id": "UNKNOWN:0002",
  "gene_symbol": "OR51G1",
  "gene": "UniProtKB:Q8NGK1",
  "term_label": "Unknown biological process",
  "gene_name": "Olfactory receptor 51G1"
}